{
  "gene_name": "Serine_threonine-protein kinase MARK1",
  "gene": "UniProtKB:Q9P0L2",
  "gene_symbol": "MARK1",
  "term_label": "intracellular signal transduction",
  "term_id": "GO:0035556"
}